{
  "gene": "UniProtKB:Q6ZN17",
  "gene_name": "Protein lin-28 homolog B",
  "gene_symbol": "LIN28B",
  "term_label": "pre-miRNA processing",
  "term_id": "GO:0031054"
}